{
  "term_label": "DNA binding",
  "gene_symbol": "H2BC1",
  "term_id": "GO:0003677",
  "gene_name": "Histone H2B type 1-A",
  "gene": "UniProtKB:Q96A08"
}